negative regulation of DNA-templated transcription initiation [GO:2000143] (biological process) Relationships: is a type of negative regulation of DNA-templated transcription [GO:0045892]; is a type of GO:2000142; negatively regulates GO:0006352 Also known as: negative regulation of DNA-dependent transcription, initiation, negative regulation of DNA-templated transcription, initiation, negative regulation of initiation of DNA-dependent transcription, negative regulation of transcription initiation, DNA-dependent Sources: GOC:mah, GOC:txnOH Definition: Any process that stops, prevents, or reduces the frequency, rate or extent of DNA-templated transcription initiation. Subtypes: GO:0060633